{
  "term_label": "nucleus",
  "gene_name": "Double homeobox protein B",
  "gene_symbol": "DUXB",
  "gene": "UniProtKB:A0A1W2PPF3",
  "term_id": "GO:0005634"
}